{
  "gene_symbol": "KLHL9",
  "gene_name": "Kelch-like protein 9",
  "term_label": "midbody",
  "gene": "UniProtKB:Q9P2J3",
  "term_id": "GO:0030496"
}